{
  "term_label": "Unknown biological process",
  "gene": "UniProtKB:P56749",
  "gene_symbol": "CLDN12",
  "term_id": "UNKNOWN:0002",
  "gene_name": "Claudin-12"
}